{
  "gene_symbol": "EBPL",
  "gene_name": "Emopamil-binding protein-like",
  "term_id": "UNKNOWN:0002",
  "gene": "UniProtKB:Q9BY08",
  "term_label": "Unknown biological process"
}